{
  "term_id": "GO:0043113",
  "gene": "UniProtKB:Q92796",
  "term_label": "receptor clustering",
  "gene_symbol": "DLG3",
  "gene_name": "Disks large homolog 3"
}